{
  "term_id": "UNKNOWN:0003",
  "gene_name": "Inositol monophosphatase 2",
  "gene_symbol": "IMPA2",
  "gene": "UniProtKB:O14732",
  "term_label": "Unknown cellular component"
}